dendritic spine [GO:0043197] (cellular component) Relationships: is a type of neuron spine [GO:0044309]; is a type of postsynapse [GO:0098794]; is part of dendrite [GO:0030425] Also known as: dendrite spine, branched dendritic spine, mushroom dendritic spine, sessile dendritic spine, stubby dendritic spine, thin dendritic spine Definition: A small, membranous protrusion from a dendrite that forms a postsynaptic compartment, typically receiving input from a single presynapse. They function as partially isolated biochemical and an electrical compartments. Spine morphology is variable:they can be thin, stubby, mushroom, or branched, with a continuum of intermediate morphologies. They typically terminate in a bulb shape, linked to the dendritic shaft by a restriction. Spine remodeling is though to be involved in synaptic plasticity. Subtypes: GO:0097464 Sources: GOC:nln